deoxycytidylate C-methyltransferase activity [GO:0050003] (molecular function) Definition: Catalysis of the reaction: 5,10-methylenetetrahydrofolate + dCMP = 2'-deoxy-5-methyl-5'-cytidylate + 7,8-dihydrofolate. Relationships: is a type of GO:0008169 Also known as: 5,10-methylenetetrahydrofolate:dCMP C-methyltransferase activity, dCMP methyltransferase activity, deoxycytidylate methyltransferase activity Sources: EC:2.1.1.54, RHEA:11568